{
  "term_id": "UNKNOWN:0003",
  "gene_symbol": "PRAP1",
  "term_label": "Unknown cellular component",
  "gene_name": "Proline-rich acidic protein 1",
  "gene": "UniProtKB:Q96NZ9"
}